protein-containing complex organization [GO:0043933] (biological process) Definition: Any process in which macromolecules aggregate, disaggregate, or are modified, resulting in the formation, disassembly, or alteration of a protein complex. Sources: GOC:mah Also known as: protein complex subunit organisation, protein complex subunit organization, cellular macromolecular complex organization, cellular macromolecular complex subunit organisation, cellular macromolecular complex subunit organization, macromolecular complex organization, macromolecular complex subunit organisation, macromolecular complex subunit organization, protein-containing complex subunit organization Relationships: is_a cellular component organization [GO:0016043] Subtypes: protein-DNA-RNA complex organization [GO:0001115], nuclear pore organization [GO:0006999], protein-containing complex disassembly [GO:0032984], GO:0034367, intermediate filament polymerization or depolymerization [GO:0045105], GO:0065003, protein-carbohydrate complex subunit organization [GO:0071823], protein-DNA complex organization [GO:0071824], protein-lipid complex organization [GO:0071825], protein-RNA complex organization [GO:0071826]